delta-type opioid receptor binding [GO:0031850] (molecular function) Relationships: is a type of opioid receptor binding [GO:0031628] Also known as: delta-type opioid receptor ligand, enkephalin receptor binding Sources: GOC:mah, GOC:nln Definition: Binding to a delta-type opioid receptor.